{
  "gene_symbol": "HECTD3",
  "gene": "UniProtKB:Q5T447",
  "term_id": "GO:0043161",
  "term_label": "proteasome-mediated ubiquitin-dependent protein catabolic process",
  "gene_name": "E3 ubiquitin-protein ligase HECTD3"
}